{
  "gene": "UniProtKB:Q8IUZ5",
  "term_id": "UNKNOWN:0001",
  "gene_name": "5-phosphohydroxy-L-lysine phospho-lyase",
  "term_label": "Unknown molecular function",
  "gene_symbol": "PHYKPL"
}